{
  "gene_symbol": "ODAD1",
  "term_id": "GO:0036158",
  "gene_name": "Outer dynein arm-docking complex subunit 1",
  "gene": "UniProtKB:Q96M63",
  "term_label": "outer dynein arm assembly"
}